{
  "term_label": "regulation of transcription by RNA polymerase II",
  "gene_symbol": "TCF23",
  "gene": "UniProtKB:Q7RTU1",
  "gene_name": "Transcription factor 23",
  "term_id": "GO:0006357"
}